{
  "term_id": "GO:0000981",
  "term_label": "DNA-binding transcription factor activity, RNA polymerase II-specific",
  "gene": "UniProtKB:Q8NHY6",
  "gene_name": "Zinc finger protein 28 homolog",
  "gene_symbol": "ZFP28"
}